{
  "gene": "UniProtKB:Q969I3",
  "term_id": "UNKNOWN:0003",
  "gene_symbol": "GLYATL1",
  "term_label": "Unknown cellular component",
  "gene_name": "Glycine N-acyltransferase-like protein 1"
}